{
  "term_id": "UNKNOWN:0001",
  "gene_name": "C-type lectin domain family 2 member L",
  "gene_symbol": "CLEC2L",
  "gene": "UniProtKB:P0C7M8",
  "term_label": "Unknown molecular function"
}